ubiquitin conjugating enzyme complex [GO:0031371] (cellular component) Also known as: E2 complex Relationships: is a type of intracellular protein-containing complex [GO:0140535]; is a type of GO:1990234 Sources: GOC:mah Subtypes: GO:0031372, HULC complex [GO:0033503], CUE1-UBC7 ubiquitin-conjugating enzyme complex [GO:1990389] Definition: Any complex that possesses ubiquitin conjugating enzyme activity.